{
  "term_label": "plasma membrane",
  "gene_name": "Olfactory receptor 4C45",
  "gene": "UniProtKB:A6NMZ5",
  "term_id": "GO:0005886",
  "gene_symbol": "OR4C45"
}